neuropeptide catabolic process [GO:0010813] (BP) Relationships: is a type of peptide catabolic process [GO:0043171] Sources: GOC:BHF, GOC:dph, GOC:tb Definition: The chemical reactions and pathways resulting in the breakdown of neuropeptides. Neuropeptides are signaling peptides that travel across a synaptic junction. Subtypes: substance P catabolic process [GO:0010814]